{
  "term_id": "GO:0005634",
  "term_label": "nucleus",
  "gene": "UniProtKB:Q6QN14",
  "gene_name": "Ubiquitin carboxyl-terminal hydrolase 17-like protein 6",
  "gene_symbol": "USP17L6P"
}